{
  "gene_symbol": "METRN",
  "gene": "UniProtKB:Q9UJH8",
  "term_label": "hormone activity",
  "gene_name": "Meteorin",
  "term_id": "GO:0005179"
}